{
  "term_id": "UNKNOWN:0002",
  "gene_symbol": "FBXO36",
  "term_label": "Unknown biological process",
  "gene": "UniProtKB:Q8NEA4",
  "gene_name": "F-box only protein 36"
}